delamination [GO:0060232] (BP) Definition: The process of negative regulation of cell adhesion that results in a cell or sheet of cells splitting off from an existing epithelial sheet. Relationships: is a type of negative regulation of cell-cell adhesion [GO:0022408] References: PMID:16962574, PMID:18343170 Sources: GOC:dph Subtypes: GO:0003336, border follicle cell delamination [GO:0030709], GO:0036032, delamination involved in gastrulation with mouth forming second [GO:0055112], oenocyte delamination [GO:0060233], GO:0060234, blood vessel endothelial cell delamination [GO:0097497], endothelial to hematopoietic transition [GO:0098508]